{
  "gene_name": "Immunoglobulin lambda variable 3-25",
  "gene_symbol": "IGLV3-25",
  "term_id": "GO:0006955",
  "term_label": "immune response",
  "gene": "UniProtKB:P01717"
}